{
  "gene_symbol": "EDA",
  "term_id": "GO:0006955",
  "term_label": "immune response",
  "gene_name": "Ectodysplasin-A",
  "gene": "UniProtKB:Q92838"
}